{
  "gene": "UniProtKB:P78412",
  "gene_symbol": "IRX6",
  "gene_name": "Iroquois-class homeodomain protein IRX-6",
  "term_label": "cell development",
  "term_id": "GO:0048468"
}